juvenile hormone metabolic process [GO:0006716] (biological process) Relationships: is a type of sesquiterpenoid metabolic process [GO:0006714]; is a type of hormone metabolic process [GO:0042445] Sources: GOC:go_curators, ISBN:0198547684 Definition: The chemical reactions and pathways involving juvenile hormones, the three sesquiterpenoid derivatives that function to maintain the larval state of insects at molting and that may be required for other processes, e.g. oogenesis. Also known as: juvenile hormone metabolism Regulation: negatively regulated by GO:0045928 Subtypes: juvenile hormone biosynthetic process [GO:0006718], juvenile hormone catabolic process [GO:0006719]